{
  "term_label": "phosphoribosylformylglycinamidine synthase activity",
  "gene": "UniProtKB:O15067",
  "term_id": "GO:0004642",
  "gene_symbol": "PFAS",
  "gene_name": "Phosphoribosylformylglycinamidine synthase"
}